ubiquitin conjugating enzyme binding [GO:0031624] (molecular function) Definition: Binding to a ubiquitin conjugating enzyme, any of the E2 proteins. Relationships: is a type of ubiquitin-like protein conjugating enzyme binding [GO:0044390] Sources: GOC:vp